structural constituent of cutaneous appendage [GO:0030281] (molecular function) Definition: The action of a molecule that contributes to the structural integrity of cutaneous epidermal structures such as hairs, scales, or feathers. Sources: GOC:mah, ISBN:0878932437 Relationships: is a type of structural molecule activity [GO:0005198]